{
  "gene_name": "Mesoderm posterior protein 1",
  "term_label": "RNA polymerase II cis-regulatory region sequence-specific DNA binding",
  "gene_symbol": "MESP1",
  "term_id": "GO:0000978",
  "gene": "UniProtKB:Q9BRJ9"
}